{
  "term_label": "regulation of apoptotic process",
  "gene_symbol": "SLK",
  "term_id": "GO:0042981",
  "gene_name": "STE20-like serine_threonine-protein kinase",
  "gene": "UniProtKB:Q9H2G2"
}